{
  "term_id": "GO:0036464",
  "term_label": "cytoplasmic ribonucleoprotein granule",
  "gene_symbol": "AGO3",
  "gene_name": "Protein argonaute-3",
  "gene": "UniProtKB:Q9H9G7"
}